{
  "term_label": "cytoplasm",
  "gene_symbol": "CDK14",
  "term_id": "GO:0005737",
  "gene_name": "Cyclin-dependent kinase 14",
  "gene": "UniProtKB:O94921"
}